{
  "term_id": "GO:0009449",
  "gene": "UniProtKB:Q99259",
  "gene_symbol": "GAD1",
  "term_label": "gamma-aminobutyric acid biosynthetic process",
  "gene_name": "Glutamate decarboxylase 1"
}